{
  "term_id": "UNKNOWN:0001",
  "gene": "UniProtKB:Q8N6Q1",
  "gene_name": "Transmembrane and coiled-coil domain-containing protein 5A",
  "gene_symbol": "TMCO5A",
  "term_label": "Unknown molecular function"
}